toxin-antitoxin complex [GO:0110001] (cellular component) Definition: A bacterial protein complex that neutralises its own toxin by complexing the toxin with the antitoxin. The antitoxin can be either a protein or an RNA. The neutralising toxin-antitoxin complex also acts as a transcriptional repressor of the toxin-antitoxin operon. Note: An example is YoeB (P69348) in Escherichia coli in PMID:16109374 (inferred by direct evidence). References: PMID:16109374, PMID:25093388 Sources: GOC:bhm Relationships: is_a GO:0017053